{
  "gene": "UniProtKB:Q569G3",
  "gene_name": "Uncharacterized protein C5orf47",
  "term_id": "UNKNOWN:0001",
  "gene_symbol": "C5orf47",
  "term_label": "Unknown molecular function"
}